sulochrin oxidase [(+)-bisdechlorogeodin-forming] activity [GO:0047064] (molecular function) Sources: EC:1.21.3.4, RHEA:24092 Also known as: sulochrin oxidase activity, sulochrin:oxygen oxidoreductase (cyclizing, (+)-specific) Definition: Catalysis of the reaction: O2 + 2 sulochrin = 2 (2S)-bisdechlorogeodin + 2 H2O. Relationships: is a type of oxidoreductase activity, acting on X-H and Y-H to form an X-Y bond, with oxygen as acceptor [GO:0046993]